{
  "term_id": "GO:0005615",
  "gene": "UniProtKB:P09486",
  "term_label": "extracellular space",
  "gene_name": "SPARC",
  "gene_symbol": "SPARC"
}